{
  "term_label": "U12-type spliceosomal complex",
  "gene_name": "Zinc finger matrin-type protein 5",
  "gene_symbol": "ZMAT5",
  "term_id": "GO:0005689",
  "gene": "UniProtKB:Q9UDW3"
}